{
  "gene": "UniProtKB:Q9NTU7",
  "gene_symbol": "CBLN4",
  "gene_name": "Cerebellin-4",
  "term_id": "GO:0043083",
  "term_label": "synaptic cleft"
}